{
  "gene_symbol": "MAP1LC3A",
  "term_id": "GO:0031625",
  "gene_name": "Microtubule-associated proteins 1A_1B light chain 3A",
  "gene": "UniProtKB:Q9H492",
  "term_label": "ubiquitin protein ligase binding"
}